(-)-E-beta-caryophyllene synthase activity [GO:0080016] (molecular function) Definition: Catalysis of the reaction: 2-trans,6-trans-farnesyl diphosphate = (-)-E-beta-caryophyllene + diphosphate. Relationships: is a type of cyclase activity [GO:0009975]; is a type of sesquiterpene synthase activity [GO:0010334] References: PMID:12566586, PMID:9442047 Sources: MetaCyc:RXN-8414